DNA topoisomerase type II (double strand cut, ATP-hydrolyzing) inhibitor activity [GO:0008657] (molecular function) Also known as: DNA gyrase inhibitor activity Relationships: is a type of enzyme inhibitor activity [GO:0004857]; is a type of ATPase inhibitor activity [GO:0042030]; is a type of DNA topoisomerase type II (double strand cut, ATP-hydrolyzing) regulator activity [GO:0072586]; negatively regulates DNA topoisomerase type II (double strand cut, ATP-hydrolyzing) activity [GO:0003918] Definition: Binds to and stops, prevents or reduces the activity of ATP-hydrolyzing DNA topoisomerase. ATP-hydrolyzing DNA topoisomerase catalyzes the DNA topological transformation by transiently cleaving a pair of complementary DNA strands to form a gate through which a second double-stranded DNA segment is passed, after which the severed strands in the first DNA segment are rejoined; product release is coupled to ATP binding and hydrolysis; changes the linking number in multiples of 2. Sources: GOC:mah